{
  "gene": "UniProtKB:P41594",
  "term_label": "regulation of synaptic transmission, glutamatergic",
  "term_id": "GO:0051966",
  "gene_symbol": "GRM5",
  "gene_name": "Metabotropic glutamate receptor 5"
}